{
  "term_id": "GO:0007096",
  "gene_name": "Dual specificity protein phosphatase CDC14C",
  "gene": "UniProtKB:A4D256",
  "gene_symbol": "CDC14C",
  "term_label": "regulation of exit from mitosis"
}